beta-carotene biosynthetic process [GO:1901812] (biological process) Definition: The chemical reactions and pathways resulting in the formation of beta-carotene. References: PMID:11387982 Sources: GOC:TermGenie, GOC:yaf, MetaCyc:PWY-5943, UniPathway:UPA00802 Also known as: beta-carotene anabolism, beta-carotene biosynthesis, beta-carotene formation, beta-carotene synthesis Relationships: is a type of carotenoid biosynthetic process [GO:0016117]; is_a carotene biosynthetic process [GO:0016120]; is a type of beta-carotene metabolic process [GO:1901810]